{
  "term_id": "GO:0051899",
  "gene": "UniProtKB:P07510",
  "term_label": "membrane depolarization",
  "gene_name": "Acetylcholine receptor subunit gamma",
  "gene_symbol": "CHRNG"
}